{
  "gene_name": "Protein arginine N-methyltransferase 9",
  "gene_symbol": "PRMT9",
  "gene": "UniProtKB:Q6P2P2",
  "term_label": "histone methyltransferase activity",
  "term_id": "GO:0042054"
}